negative regulation of the force of heart contraction by chemical signal [GO:0003108] (biological process) Subtypes: negative regulation of the force of heart contraction by acetylcholine [GO:0003060] Definition: Any process which decreases the force of heart muscle contraction mediated by chemical signaling, hormonal, autocrine or paracrine. Also known as: negative regulation of the force of heart muscle contraction by chemical signal Sources: GOC:mtg_cardio Relationships: is a type of regulation of the force of heart contraction by chemical signal [GO:0003057]; is a type of GO:0045822